{
  "term_label": "Unknown molecular function",
  "gene_symbol": "ADAMTSL1",
  "gene": "UniProtKB:Q8N6G6",
  "term_id": "UNKNOWN:0001",
  "gene_name": "ADAMTS-like protein 1"
}